response to D-galactose [GO:1905377] (biological process) Definition: Any process that results in a change in state or activity of a cell or an organism (in terms of movement, secretion, enzyme production, gene expression, etc.) as a result of a D-galactose stimulus. References: PMID:26261574 Sources: GOC:TermGenie, GO_REF:0000071 Relationships: is a type of response to hexose [GO:0009746] Also known as: response to D-Gal, response to D-galacto-hexose Subtypes: cellular response to D-galactose [GO:1905378]